substance P receptor activity [GO:0016496] (molecular function) Definition: Combining with substance P, the peptide Arg-Pro-Lys-Pro-Gln-Gln-Phe-Phe-Gly-Leu-Met, to initiate a change in cell activity. Relationships: is a type of tachykinin receptor activity [GO:0004995] Sources: GOC:mah, ISBN:0198506732